cyanogenic glycoside biosynthetic process [GO:0019756] (BP) Sources: ISBN:0198506732 Subtypes: dhurrin biosynthetic process [GO:0010132], 4-hydroxyindole-3- carbonyl nitrile biosynthesis [GO:0106148] Definition: The chemical reactions and pathways resulting in the formation of cyanogenic glycosides, any glycoside containing a cyano group that is released as hydrocyanic acid on acid hydrolysis; such compounds occur in the kernels of various fruits. Also known as: cyanogenic glycoside anabolism, cyanogenic glycoside biosynthesis, cyanogenic glycoside formation, cyanogenic glycoside synthesis Relationships: is a type of glycoside biosynthetic process [GO:0016138]; is a type of GO:0044550; is a type of GO:0080028